{
  "gene_symbol": "H2AC8",
  "term_id": "GO:0031507",
  "term_label": "heterochromatin formation",
  "gene_name": "Histone H2A type 1-B_E",
  "gene": "UniProtKB:P04908"
}